regulation of pyrimidine nucleoside transport [GO:0032246] (BP) Relationships: is a type of regulation of nucleoside transport [GO:0032242]; regulates pyrimidine nucleoside transport [GO:0015864] Definition: Any process that modulates the frequency, rate or extent of the directed movement of a pyrimidine nucleoside into, out of or within a cell, or between cells, by means of some agent such as a transporter or pore. Sources: GOC:mah